{
  "gene": "UniProtKB:Q92835",
  "gene_symbol": "INPP5D",
  "term_label": "cytosol",
  "gene_name": "Phosphatidylinositol 3,4,5-trisphosphate 5-phosphatase 1",
  "term_id": "GO:0005829"
}